{
  "gene_name": "Phosphatidylinositol 5-phosphate 4-kinase type-2 alpha",
  "gene_symbol": "PIP4K2A",
  "gene": "UniProtKB:P48426",
  "term_label": "plasma membrane",
  "term_id": "GO:0005886"
}